{
  "term_label": "extracellular space",
  "gene": "UniProtKB:O75636",
  "gene_name": "Ficolin-3",
  "term_id": "GO:0005615",
  "gene_symbol": "FCN3"
}